{
  "term_id": "GO:0005518",
  "gene": "UniProtKB:Q16832",
  "gene_name": "Discoidin domain-containing receptor 2",
  "term_label": "collagen binding",
  "gene_symbol": "DDR2"
}